{
  "term_label": "mitochondrial mRNA catabolic process",
  "gene_name": "Polyribonucleotide nucleotidyltransferase 1, mitochondrial",
  "gene_symbol": "PNPT1",
  "term_id": "GO:0000958",
  "gene": "UniProtKB:Q8TCS8"
}